{
  "gene_name": "Mu-type opioid receptor",
  "term_label": "neuron projection",
  "gene_symbol": "OPRM1",
  "gene": "UniProtKB:P35372",
  "term_id": "GO:0043005"
}